{
  "term_id": "GO:0000976",
  "gene": "UniProtKB:Q4LE39",
  "gene_symbol": "ARID4B",
  "term_label": "transcription cis-regulatory region binding",
  "gene_name": "AT-rich interactive domain-containing protein 4B"
}